peptidyl-lysine deglycation [GO:0036528] (biological process) Definition: The removal of a sugar or dicarbonyl from a lysine residue of a glycated protein. Relationships: is a type of peptidyl-lysine modification [GO:0018205]; is a type of protein deglycation [GO:0036525] References: PMID:14568004, PMID:25416785 Sources: GOC:PARL, GOC:bf Also known as: deglycation of N-acetyllysine